{
  "gene": "UniProtKB:Q9BQ95",
  "term_id": "GO:0060090",
  "gene_symbol": "ECSIT",
  "term_label": "molecular adaptor activity",
  "gene_name": "Evolutionarily conserved signaling intermediate in Toll pathway, mitochondrial"
}